{
  "gene_symbol": "IGSF5",
  "gene": "UniProtKB:Q9NSI5",
  "term_label": "cell surface",
  "term_id": "GO:0009986",
  "gene_name": "Immunoglobulin superfamily member 5"
}